{
  "gene_name": "Protein phosphatase 1 regulatory subunit 21",
  "term_label": "Unknown molecular function",
  "gene_symbol": "PPP1R21",
  "gene": "UniProtKB:Q6ZMI0",
  "term_id": "UNKNOWN:0001"
}